positive regulation of phosphate metabolic process [GO:0045937] (biological process) Relationships: is a type of positive regulation of phosphorus metabolic process [GO:0010562]; positively regulates GO:0006796 Subtypes: positive regulation of dephosphorylation [GO:0035306], positive regulation of phosphorylation [GO:0042327], positive regulation of nucleotide metabolic process [GO:0045981], positive regulation of fructose 1,6-bisphosphate metabolic process [GO:0060552], GO:0060732, GO:0106280, positive regulation of pyruvate decarboxylation to acetyl-CoA [GO:0140176], positive regulation of butyryl-CoA biosynthetic process from acetyl-CoA [GO:1900496], positive regulation of butyryl-CoA catabolic process to butanol [GO:1900499], positive regulation of butyryl-CoA catabolic process to butyrate [GO:1900502], positive regulation of sarcinapterin biosynthetic process [GO:1900973], positive regulation of tetrapyrrole biosynthetic process from glycine and succinyl-CoA [GO:1901415], GO:1903727 Sources: GOC:go_curators Also known as: positive regulation of phosphate metabolism, up regulation of phosphate metabolic process, up-regulation of phosphate metabolic process, upregulation of phosphate metabolic process, activation of phosphate metabolic process, stimulation of phosphate metabolic process Definition: Any process that activates or increases the frequency, rate or extent of the chemical reactions and pathways involving phosphates.